{
  "term_id": "GO:0016887",
  "gene_symbol": "ATAD2",
  "gene_name": "ATPase family AAA domain-containing protein 2",
  "gene": "UniProtKB:Q6PL18",
  "term_label": "ATP hydrolysis activity"
}